{
  "gene_symbol": "DFFA",
  "gene": "UniProtKB:O00273",
  "gene_name": "DNA fragmentation factor subunit alpha",
  "term_label": "negative regulation of apoptotic DNA fragmentation",
  "term_id": "GO:1902511"
}